{
  "gene": "UniProtKB:Q8WTT2",
  "term_id": "GO:0005730",
  "term_label": "nucleolus",
  "gene_name": "Nucleolar complex protein 3 homolog",
  "gene_symbol": "NOC3L"
}